{
  "term_label": "nucleus",
  "term_id": "GO:0005634",
  "gene": "UniProtKB:A0A024RBG1",
  "gene_name": "Diphosphoinositol polyphosphate phosphohydrolase NUDT4B",
  "gene_symbol": "NUDT4B"
}